{
  "gene": "UniProtKB:P01275",
  "term_id": "GO:0007188",
  "gene_symbol": "GCG",
  "gene_name": "Pro-glucagon",
  "term_label": "adenylate cyclase-modulating G protein-coupled receptor signaling pathway"
}